{
  "gene_name": "NADH dehydrogenase [ubiquinone] 1 alpha subcomplex assembly factor 3",
  "term_label": "mitochondrial inner membrane",
  "gene_symbol": "NDUFAF3",
  "gene": "UniProtKB:Q9BU61",
  "term_id": "GO:0005743"
}